{
  "term_label": "DNA-binding transcription factor activity, RNA polymerase II-specific",
  "gene": "UniProtKB:Q68CJ9",
  "term_id": "GO:0000981",
  "gene_name": "Cyclic AMP-responsive element-binding protein 3-like protein 3",
  "gene_symbol": "CREB3L3"
}